C-8 sterol isomerase activity [GO:0000247] (molecular function) Definition: Catalysis of the reaction: fecosterol = episterol. References: PMID:8988026 Sources: RHEA:33435 Relationships: is a type of GO:0016863 Also known as: delta-8-delta-7 sterol isomerase activity